{
  "gene_name": "Zinc finger protein 713",
  "gene": "UniProtKB:Q8N859",
  "gene_symbol": "ZNF713",
  "term_id": "GO:0000981",
  "term_label": "DNA-binding transcription factor activity, RNA polymerase II-specific"
}